{
  "gene": "UniProtKB:Q5TAA0",
  "gene_name": "Tetratricopeptide repeat protein 22",
  "gene_symbol": "TTC22",
  "term_label": "Unknown molecular function",
  "term_id": "UNKNOWN:0001"
}